developmental cell growth [GO:0048588] (biological process) Definition: The growth of a cell, where growth contributes to the progression of the cell over time from one condition to another. Sources: GOC:go_curators, GOC:isa_complete Also known as: developmental growth of a unicellular organism Relationships: is a type of GO:0016049; is a type of developmental growth [GO:0048589]; is part of cell development [GO:0048468] Subtypes: oocyte growth [GO:0001555], post-embryonic cardiac muscle cell growth involved in heart morphogenesis [GO:0003247], chondrocyte hypertrophy [GO:0003415], primary spermatocyte growth [GO:0007285], pollen tube growth [GO:0009860], glial cell growth [GO:0042065], collateral sprouting [GO:0048668], GO:0048682, root hair elongation [GO:0048767], cell growth involved in cardiac muscle cell development [GO:0061049], cell growth involved in Malpighian tubule morphogenesis [GO:0061335], neuron projection extension [GO:1990138]